protein folding in endoplasmic reticulum [GO:0034975] (biological process) Definition: A protein folding process that takes place in the endoplasmic reticulum (ER). Secreted, plasma membrane and organelle proteins are folded in the ER, assisted by chaperones and foldases (protein disulphide isomerases), and additional factors required for optimal folding (ATP, Ca2+ and an oxidizing environment to allow disulfide bond formation). Sources: GOC:mah, GOC:vw Also known as: oxidative protein folding, protein folding in ER Relationships: is a type of protein folding [GO:0006457] Regulation: regulated by GO:0060904